cellular response to menadione [GO:0036245] (biological process) Sources: GOC:al, Wikipedia:Menadione Also known as: cellular response to vitamin K3 Definition: Any process that results in a change in state or activity of a cell (in terms of movement, secretion, enzyme production, gene expression, etc.) as a result of a menadione stimulus. Menadione (also called vitamin K3) is a naphthoquinone having a methyl substituent at the 2-position. Relationships: is a type of cellular response to vitamin K [GO:0071307]